{
  "term_label": "Golgi membrane",
  "term_id": "GO:0000139",
  "gene_name": "Furin",
  "gene_symbol": "FURIN",
  "gene": "UniProtKB:P09958"
}